{
  "gene_name": "Galactosylgalactosylxylosylprotein 3-beta-glucuronosyltransferase 1",
  "term_label": "galactosylgalactosylxylosylprotein 3-beta-glucuronosyltransferase activity",
  "term_id": "GO:0015018",
  "gene": "UniProtKB:Q9P2W7",
  "gene_symbol": "B3GAT1"
}